{
  "gene_symbol": "SMURF2",
  "term_label": "proteasome-mediated ubiquitin-dependent protein catabolic process",
  "gene_name": "E3 ubiquitin-protein ligase SMURF2",
  "term_id": "GO:0043161",
  "gene": "UniProtKB:Q9HAU4"
}